Myc-Max complex [GO:0071943] (cellular component) Relationships: is a type of RNA polymerase II transcription regulator complex [GO:0090575] Definition: A transcription factor complex that consists of a heterodimer of the bHLH-ZIP proteins Myc and Max. References: PMID:16620027, PMID:16620031, PMID:20170194 Sources: GOC:cna